{
  "term_id": "GO:0016020",
  "term_label": "membrane",
  "gene_symbol": "TMEM86A",
  "gene": "UniProtKB:Q8N2M4",
  "gene_name": "Lysoplasmalogenase-like protein TMEM86A"
}